dethiobiotin synthase activity [GO:0004141] (molecular function) Definition: Catalysis of the reaction: 7,8-diaminononanoate + ATP + CO2 = ADP + dethiobiotin + 4 H+ + phosphate. Also known as: 7,8-diaminononanoate:carbon-dioxide cyclo-ligase (ADP-forming), DTB synthetase activity, desthiobiotin synthase activity Sources: EC:6.3.3.3, RHEA:15805 Relationships: is a type of cyclo-ligase activity [GO:0016882]